{
  "gene": "UniProtKB:P13866",
  "term_label": "renal D-glucose absorption",
  "gene_symbol": "SLC5A1",
  "term_id": "GO:0035623",
  "gene_name": "Sodium_glucose cotransporter 1"
}